effector-mediated perturbation of host defenses by symbiont [GO:0140415] (biological process) Definition: A process mediated by a molecule secreted by a symbiont that results in the modulation (either activation or suppression) of a defense response. The host is defined as the larger of the organisms involved in a symbiotic interaction. References: PMID:30610168 Also known as: effector-mediated modulation of host defenses by symbiont Relationships: is a type of symbiont-mediated perturbation of host defense response [GO:0052031]; is a type of symbiont-mediated response to host defenses [GO:0052200]; is a type of effector-mediated perturbation of host process by symbiont [GO:0140418] Subtypes: effector-mediated perturbation of host innate immune response by symbiont [GO:0140404], GO:0140590